{
  "gene": "UniProtKB:Q8TAK5",
  "gene_name": "GA-binding protein subunit beta-2",
  "term_id": "GO:0045944",
  "gene_symbol": "GABPB2",
  "term_label": "positive regulation of transcription by RNA polymerase II"
}